phorbol ester receptor activity [GO:0001565] (molecular function) Relationships: is a type of GO:0038023 Subtypes: non-kinase phorbol ester receptor activity [GO:0001566] Definition: Combining with a phorbol ester and transmitting the signal to initiate a change in cell activity. References: PMID:10506570 Sources: GOC:ai, GOC:signaling